{
  "gene_symbol": "MRPS23",
  "gene_name": "Small ribosomal subunit protein mS23",
  "gene": "UniProtKB:Q9Y3D9",
  "term_id": "UNKNOWN:0001",
  "term_label": "Unknown molecular function"
}